{
  "gene_name": "Transcription factor IIIA",
  "gene": "UniProtKB:Q92664",
  "term_id": "UNKNOWN:0002",
  "gene_symbol": "GTF3A",
  "term_label": "Unknown biological process"
}